{
  "term_label": "transcription coactivator activity",
  "gene_symbol": "SUB1",
  "gene": "UniProtKB:P53999",
  "gene_name": "Activated RNA polymerase II transcriptional coactivator p15",
  "term_id": "GO:0003713"
}